{
  "term_label": "endoplasmic reticulum",
  "gene_name": "Protein phosphatase 1 regulatory subunit 15B",
  "term_id": "GO:0005783",
  "gene_symbol": "PPP1R15B",
  "gene": "UniProtKB:Q5SWA1"
}